{
  "gene": "UniProtKB:Q99928",
  "term_id": "GO:0022851",
  "term_label": "GABA-gated chloride ion channel activity",
  "gene_name": "Gamma-aminobutyric acid receptor subunit gamma-3",
  "gene_symbol": "GABRG3"
}